response to glyceraldehyde [GO:1905630] (biological process) References: PMID:11377826 Sources: GOC:TermGenie, GO_REF:0000071 Subtypes: cellular response to glyceraldehyde [GO:1905631] Relationships: is a type of response to monosaccharide [GO:0034284] Definition: Any process that results in a change in state or activity of a cell or an organism (in terms of movement, secretion, enzyme production, gene expression, etc.) as a result of a glyceraldehyde stimulus.